sulfate assimilation via adenylyl sulfate reduction [GO:0010134] (BP) Relationships: is a type of sulfate assimilation [GO:0000103]; has part adenylyl-sulfate reductase activity [GO:0009973] Sources: MetaCyc:SULFMETII-PWY Also known as: sulphate assimilation via adenylyl sulphate reduction Definition: The pathway by which inorganic sulfate is activated, reduced and incorporated into sulfated compounds, where the activated sulfate, adenylyl-sulfate, is reduced to sulfite by the activity of adenylyl-sulfate reductase.